{
  "gene": "UniProtKB:Q9Y5X0",
  "term_id": "GO:1901981",
  "gene_name": "Sorting nexin-10",
  "gene_symbol": "SNX10",
  "term_label": "phosphatidylinositol phosphate binding"
}